{
  "gene": "UniProtKB:Q9NRI7",
  "term_id": "UNKNOWN:0002",
  "gene_name": "Putative pancreatic polypeptide 2",
  "term_label": "Unknown biological process",
  "gene_symbol": "PPY2P"
}